{
  "term_label": "histone H3K9 methyltransferase activity",
  "gene_name": "Histone-lysine N-methyltransferase EHMT2",
  "gene_symbol": "EHMT2",
  "term_id": "GO:0046974",
  "gene": "UniProtKB:Q96KQ7"
}